{
  "term_label": "Unknown cellular component",
  "term_id": "UNKNOWN:0003",
  "gene_name": "Protein FAM43B",
  "gene_symbol": "FAM43B",
  "gene": "UniProtKB:Q6ZT52"
}